{
  "term_label": "plasma membrane",
  "gene": "UniProtKB:Q9H2B2",
  "gene_name": "Synaptotagmin-4",
  "term_id": "GO:0005886",
  "gene_symbol": "SYT4"
}